natural killer cell mediated immune response to tumor cell [GO:0002423] (biological process) Definition: An immune response mediated by a natural killer cell triggered in response to the presence of a tumor cell. Regulation: RO_0002211 by regulation of natural killer cell mediated immune response to tumor cell [GO:0002855]; negatively regulated by negative regulation of natural killer cell mediated immune response to tumor cell [GO:0002856]; positively regulated by positive regulation of natural killer cell mediated immune response to tumor cell [GO:0002857] Subtypes: GO:0002420 Relationships: is a type of natural killer cell mediated immunity [GO:0002228]; is a type of GO:0002418 References: PMID:16730260 Sources: GOC:add, ISBN:0781735149